{
  "gene": "UniProtKB:P28335",
  "term_label": "serotonin receptor signaling pathway",
  "gene_symbol": "HTR2C",
  "term_id": "GO:0007210",
  "gene_name": "5-hydroxytryptamine receptor 2C"
}